positive regulation of viral process [GO:0048524] (biological process) Definition: Any process that activates or increases the frequency, rate or extent of a multi-organism process in which a virus is a participant. Sources: GOC:bf, GOC:jl Also known as: activation of viral life cycle, positive regulation of viral life cycle, positive regulation of viral reproduction, stimulation of viral life cycle, up regulation of viral life cycle, up-regulation of viral life cycle, upregulation of viral life cycle Relationships: is_a positive regulation of biological process [GO:0048518]; is a type of regulation of viral process [GO:0050792]; positively regulates viral process [GO:0016032] Subtypes: positive regulation of viral genome replication [GO:0045070], positive regulation by virus of viral protein levels in host cell [GO:0046726], GO:0050434, positive regulation of viral life cycle [GO:1903902], positive regulation of viral translation [GO:1904973]